{
  "term_id": "GO:0043029",
  "term_label": "T cell homeostasis",
  "gene_symbol": "PPP2R3C",
  "gene_name": "Serine_threonine-protein phosphatase 2A regulatory subunit B'' subunit gamma",
  "gene": "UniProtKB:Q969Q6"
}